{
  "gene": "UniProtKB:Q5VZ18",
  "gene_name": "SH2 domain-containing adapter protein E",
  "term_id": "UNKNOWN:0002",
  "gene_symbol": "SHE",
  "term_label": "Unknown biological process"
}